{
  "term_id": "UNKNOWN:0001",
  "gene": "UniProtKB:A0A075B7B9",
  "gene_name": "Protein IGHD2OR15-2A (Fragment)",
  "gene_symbol": "IGHD2OR15-2B",
  "term_label": "Unknown molecular function"
}